{
  "gene": "UniProtKB:P32970",
  "gene_symbol": "CD70",
  "gene_name": "CD70 antigen",
  "term_id": "UNKNOWN:0002",
  "term_label": "Unknown biological process"
}